{
  "gene_symbol": "GTF2A1L",
  "term_id": "UNKNOWN:0001",
  "gene": "UniProtKB:Q9UNN4",
  "gene_name": "TFIIA-alpha and beta-like factor",
  "term_label": "Unknown molecular function"
}